9beta-pimara-7,15-diene oxidase activity [GO:0036209] (molecular function) Also known as: 9-beta-stemod-13(17)-ene oxidase activity Sources: RHEA:31951 Definition: Catalysis of the reaction: 9beta-pimara-7,15-diene + 3 O2 + 3 reduced [NADPH-hemoprotein reductase] = 9beta-pimara-7,15-dien-19-oate + 4 H+ + 4 H2O + 3 oxidized [NADPH-hemoprotein reductase]. Relationships: is a type of GO:0016709